{
  "gene": "UniProtKB:Q92995",
  "term_id": "GO:0004843",
  "gene_symbol": "USP13",
  "term_label": "cysteine-type deubiquitinase activity",
  "gene_name": "Ubiquitin carboxyl-terminal hydrolase 13"
}